{
  "gene": "UniProtKB:P09038",
  "gene_name": "Fibroblast growth factor 2",
  "gene_symbol": "FGF2",
  "term_label": "positive regulation of cell population proliferation",
  "term_id": "GO:0008284"
}